{
  "gene_symbol": "ZNF709",
  "term_id": "GO:0000977",
  "gene": "UniProtKB:Q8N972",
  "term_label": "RNA polymerase II transcription regulatory region sequence-specific DNA binding",
  "gene_name": "Zinc finger protein 709"
}